{
  "gene": "UniProtKB:O00445",
  "term_label": "calcium-dependent phospholipid binding",
  "gene_name": "Synaptotagmin-5",
  "gene_symbol": "SYT5",
  "term_id": "GO:0005544"
}